{
  "term_label": "triglyceride homeostasis",
  "term_id": "GO:0070328",
  "gene_name": "Angiopoietin-related protein 4",
  "gene_symbol": "ANGPTL4",
  "gene": "UniProtKB:Q9BY76"
}